negative regulation of stress granule assembly [GO:0062030] (BP) Relationships: is a type of GO:0062028; is a type of negative regulation of organelle assembly [GO:1902116]; negatively regulates stress granule assembly [GO:0034063] References: PMID:20180778 Definition: Any process that stops or decreases the rate, frequency or extent of stress-granule assembly, the aggregation, arrangement and bonding together of proteins and RNA molecules to form a stress granule.